{
  "term_label": "positive regulation of gluconeogenesis",
  "gene_symbol": "PRKAG1",
  "gene_name": "5'-AMP-activated protein kinase subunit gamma-1",
  "gene": "UniProtKB:P54619",
  "term_id": "GO:0045722"
}